positive regulation of growth hormone receptor signaling pathway [GO:0060399] (biological process) Relationships: is a type of positive regulation of signal transduction [GO:0009967]; is a type of regulation of growth hormone receptor signaling pathway [GO:0060398]; positively regulates growth hormone receptor signaling pathway [GO:0060396] Definition: Any process that increases the rate, frequency or extent of the growth hormone receptor signaling pathway. The growth hormone receptor signaling pathway is the series of molecular signals generated as a consequence of growth hormone receptor binding to its physiological ligand. Sources: GOC:BHF, GOC:dph Also known as: positive regulation of growth hormone receptor signalling pathway